{
  "gene_name": "V-set and immunoglobulin domain-containing protein 10-like 2",
  "gene_symbol": "VSIG10L2",
  "term_label": "cell adhesion molecule binding",
  "gene": "UniProtKB:P0DP72",
  "term_id": "GO:0050839"
}